{
  "term_id": "UNKNOWN:0003",
  "term_label": "Unknown cellular component",
  "gene_name": "Uncharacterized protein C6orf62",
  "gene": "UniProtKB:Q9GZU0",
  "gene_symbol": "C6orf62"
}